{
  "gene": "UniProtKB:Q9NTJ4",
  "term_id": "UNKNOWN:0003",
  "gene_name": "Alpha-mannosidase 2C1",
  "term_label": "Unknown cellular component",
  "gene_symbol": "MAN2C1"
}